{
  "term_id": "GO:0003697",
  "gene_name": "ATPase SWSAP1",
  "gene_symbol": "SWSAP1",
  "term_label": "single-stranded DNA binding",
  "gene": "UniProtKB:Q6NVH7"
}